regulation of transcription from RNA polymerase II promoter by a nonfermentable carbon source [GO:0061413] (biological process) Subtypes: positive regulation of transcription from RNA polymerase II promoter by a nonfermentable carbon source [GO:0061414], negative regulation of transcription from RNA polymerase II promoter by a nonfermentable carbon source [GO:0061415] References: PMID:19686338 Sources: GOC:dph Definition: A transcription regulation process in which the presence of a nonfermentable carbon source leads to the modulation of the frequency, rate, or extent of transcription, from an RNA polymerase II promoter, of specific genes involved in the metabolism of other carbon sources. Relationships: is a type of GO:0000429